{
  "gene_name": "E3 ubiquitin-protein ligase UBR5",
  "term_label": "nucleus",
  "gene": "UniProtKB:O95071",
  "term_id": "GO:0005634",
  "gene_symbol": "UBR5"
}